{
  "gene_symbol": "PDE4B",
  "term_label": "negative regulation of cAMP/PKA signal transduction",
  "term_id": "GO:0141162",
  "gene": "UniProtKB:Q07343",
  "gene_name": "cAMP-specific 3',5'-cyclic phosphodiesterase 4B"
}